{
  "term_id": "GO:0007283",
  "gene": "UniProtKB:Q96LK8",
  "term_label": "spermatogenesis",
  "gene_symbol": "SPATA32",
  "gene_name": "Spermatogenesis-associated protein 32"
}